{
  "gene_name": "Structural maintenance of chromosomes flexible hinge domain-containing protein 1",
  "term_label": "Barr body",
  "gene_symbol": "SMCHD1",
  "gene": "UniProtKB:A6NHR9",
  "term_id": "GO:0001740"
}